{
  "gene_name": "DNA transposase THAP9",
  "term_id": "GO:0006313",
  "gene_symbol": "THAP9",
  "term_label": "DNA transposition",
  "gene": "UniProtKB:Q9H5L6"
}